germacradienol synthase activity [GO:0034004] (molecular function) Definition: Catalysis of the reaction: 2-trans,6-trans-farnesyl diphosphate + H2O = (1E,4S,5E,7R)-germacra-1(10),5-dien-11-ol + diphosphate. Also known as: 2-trans,6-trans-farnesyl-diphosphate diphosphate-lyase [(1E,4S,5E,7R)-germacra-1(10),5-dien-11-ol-forming] activity Sources: EC:4.2.3.22 Relationships: is_a GO:0016838